{
  "term_id": "GO:0070374",
  "gene": "UniProtKB:Q9ULP0",
  "gene_symbol": "NDRG4",
  "term_label": "positive regulation of ERK1 and ERK2 cascade",
  "gene_name": "Protein NDRG4"
}